{
  "gene_symbol": "ESPL1",
  "gene_name": "Separin",
  "term_label": "cysteine-type endopeptidase activity",
  "term_id": "GO:0004197",
  "gene": "UniProtKB:Q14674"
}